{
  "term_id": "GO:0005737",
  "term_label": "cytoplasm",
  "gene_name": "Toll-interacting protein",
  "gene_symbol": "TOLLIP",
  "gene": "UniProtKB:Q9H0E2"
}